{
  "gene_symbol": "ACSL6",
  "term_id": "GO:0001676",
  "term_label": "long-chain fatty acid metabolic process",
  "gene_name": "Long-chain-fatty-acid--CoA ligase 6",
  "gene": "UniProtKB:Q9UKU0"
}